positive regulation of axon regeneration [GO:0048680] (biological process) Sources: GOC:dgh, GOC:dph, GOC:jid, GOC:lm Relationships: is a type of positive regulation of response to external stimulus [GO:0032103]; is a type of regulation of axon regeneration [GO:0048679]; is a type of positive regulation of neuron projection regeneration [GO:0070572]; is_a positive regulation of response to wounding [GO:1903036]; positively regulates axon regeneration [GO:0031103] Also known as: up regulation of axon regeneration, up-regulation of axon regeneration, upregulation of axon regeneration, activation of axon regeneration, stimulation of axon regeneration Definition: Any process that activates, maintains or increases the rate of axon regeneration. Subtypes: positive regulation of collateral sprouting of intact axon in response to injury [GO:0048684], positive regulation of sprouting of injured axon [GO:0048687], positive regulation of optical nerve axon regeneration [GO:1905593]